{
  "gene_symbol": "DNAJB9",
  "term_id": "GO:0051087",
  "term_label": "protein-folding chaperone binding",
  "gene": "UniProtKB:Q9UBS3",
  "gene_name": "DnaJ homolog subfamily B member 9"
}